{
  "term_label": "proteolysis",
  "gene_name": "Tripeptidyl-peptidase 1",
  "gene_symbol": "TPP1",
  "term_id": "GO:0006508",
  "gene": "UniProtKB:O14773"
}